{
  "term_label": "cell migration",
  "gene_symbol": "GPC4",
  "term_id": "GO:0016477",
  "gene": "UniProtKB:O75487",
  "gene_name": "Glypican-4"
}